{
  "gene_name": "Ras-related protein Rap-2a",
  "gene": "UniProtKB:P10114",
  "term_label": "plasma membrane",
  "gene_symbol": "RAP2A",
  "term_id": "GO:0005886"
}